{
  "gene_symbol": "OR5P2",
  "term_id": "GO:0005549",
  "gene_name": "Olfactory receptor 5P2",
  "term_label": "odorant binding",
  "gene": "UniProtKB:Q8WZ92"
}